{
  "gene": "UniProtKB:Q96CP2",
  "term_label": "Unknown cellular component",
  "gene_name": "FLYWCH family member 2",
  "gene_symbol": "FLYWCH2",
  "term_id": "UNKNOWN:0003"
}